{
  "gene": "UniProtKB:P39060",
  "gene_symbol": "COL18A1",
  "term_label": "extracellular matrix organization",
  "gene_name": "Collagen alpha-1(XVIII) chain",
  "term_id": "GO:0030198"
}